{
  "term_id": "GO:0016887",
  "term_label": "ATP hydrolysis activity",
  "gene_name": "Dynein regulatory complex protein 11",
  "gene_symbol": "IQCA1",
  "gene": "UniProtKB:Q86XH1"
}